{
  "gene": "UniProtKB:Q96IS3",
  "term_label": "regulation of transcription by RNA polymerase II",
  "gene_name": "Retina and anterior neural fold homeobox protein 2",
  "gene_symbol": "RAX2",
  "term_id": "GO:0006357"
}